catecholamine uptake involved in synaptic transmission [GO:0051934] (biological process) Definition: The uptake of catecholamine neurotransmitters by neurons or glial cells. This process leads to inactivation and recycling of neurotransmitters. Regulation: regulated by regulation of catecholamine uptake involved in synaptic transmission [GO:0051940]; positively regulated by positive regulation of catecholamine uptake involved in synaptic transmission [GO:0051944]; negatively regulated by negative regulation of catecholamine uptake involved in synaptic transmission [GO:0051945] Also known as: catecholamine neurotransmitter recycling, catecholamine neurotransmitter reuptake, catecholamine neurotransmitter import into glial cell, catecholamine neurotransmitter import into neuron, catecholamine reuptake during transmission of nerve impulse, catecholamine uptake during transmission of nerve impulse Sources: ISBN:0123668387 Subtypes: dopamine uptake involved in synaptic transmission [GO:0051583] Relationships: is_a catecholamine uptake [GO:0090493]; is a type of GO:0098810